{
  "gene": "UniProtKB:Q13342",
  "term_label": "DNA-binding transcription factor activity, RNA polymerase II-specific",
  "gene_name": "Nuclear body protein SP140",
  "gene_symbol": "SP140",
  "term_id": "GO:0000981"
}